{
  "gene_name": "Retinoic acid receptor RXR-alpha",
  "term_id": "GO:0030154",
  "term_label": "cell differentiation",
  "gene_symbol": "RXRA",
  "gene": "UniProtKB:P19793"
}